nucleate erythrocyte differentiation [GO:0043363] (biological process) Definition: The process in which a myeloid precursor cell acquires specializes features of an erythrocyte with a nucleus, as found in non-mammalian vertebrates such as birds. Relationships: is a type of erythrocyte differentiation [GO:0030218] Also known as: nucleate RBC differentiation, nucleate red blood cell differentiation Sources: GOC:jl